{
  "gene_name": "NAD-capped RNA hydrolase NUDT12",
  "term_label": "NADP+ catabolic process",
  "gene_symbol": "NUDT12",
  "term_id": "GO:0006742",
  "gene": "UniProtKB:Q9BQG2"
}